{
  "gene": "UniProtKB:Q15527",
  "term_label": "Unknown biological process",
  "term_id": "UNKNOWN:0002",
  "gene_name": "Surfeit locus protein 2",
  "gene_symbol": "SURF2"
}